{
  "gene_name": "Microtubule-actin cross-linking factor 1, isoforms 1_2_3_4_5",
  "term_id": "GO:0016020",
  "term_label": "membrane",
  "gene_symbol": "MACF1",
  "gene": "UniProtKB:Q9UPN3"
}